racemase and epimerase activity, acting on carbohydrates and derivatives [GO:0016857] (molecular function) Subtypes: GO:0003974, GO:0003978, aldose 1-epimerase activity [GO:0004034], D-ribulose-phosphate 3-epimerase activity [GO:0004750], GO:0008712, L-ribulose-phosphate 4-epimerase activity [GO:0008742], UDP-N-acetylglucosamine 2-epimerase activity [GO:0008761], dTDP-4-dehydrorhamnose 3,5-epimerase activity [GO:0008830], UDP-4-keto-6-deoxy-glucose-3,5-epimerase activity [GO:0010489], GO:0034015, allulose 6-phosphate 3-epimerase activity [GO:0034700], L-fucose mutarotase activity [GO:0036373], heparosan-N-sulfate-glucuronate 5-epimerase activity [GO:0047464], N-acylglucosamine-6-phosphate 2-epimerase activity [GO:0047465], GO:0047732, cellobiose epimerase activity [GO:0047736], chondroitin-glucuronate 5-epimerase activity [GO:0047757], GDP-mannose 3,5-epimerase activity [GO:0047918], glucose-6-phosphate 1-epimerase activity [GO:0047938], N-acylglucosamine 2-epimerase activity [GO:0050121], UDP-arabinose 4-epimerase activity [GO:0050373], GO:0050376, UDP-glucuronate 4-epimerase activity [GO:0050378], UDP-glucuronate 5'-epimerase activity [GO:0050379], maltose epimerase activity [GO:0050558], L-rhamnose mutarotase activity [GO:0062192] Relationships: is a type of racemase and epimerase activity [GO:0016854] Sources: EC:5.1.3.-, GOC:mah Definition: Catalysis of a reaction that alters the configuration of one or more chiral centers in a carbohydrate molecule.